{
  "gene_name": "Amidophosphoribosyltransferase",
  "gene": "UniProtKB:Q06203",
  "gene_symbol": "PPAT",
  "term_label": "Unknown cellular component",
  "term_id": "UNKNOWN:0003"
}